arabinose catabolic process [GO:0019568] (biological process) Also known as: arabinose breakdown, arabinose catabolism, arabinose degradation Subtypes: GO:0019571, GO:0019572 Sources: GOC:ai Definition: The chemical reactions and pathways resulting in the breakdown of arabinose, arabino-pentose. Relationships: is a type of pentose catabolic process [GO:0019323]; is a type of GO:0019566